metanephric late distal convoluted tubule development [GO:0072225] (biological process) Sources: GOC:mtg_kidney_jan10 Definition: The process whose specific outcome is the progression of the metanephric late distal convoluted tubule over time, from its formation to the mature structure. The metanephric late distal convoluted tubule contains metanephric DCT cells and intercalated (IC) alpha and beta cells and is vasopressin-sensitive. Relationships: is a type of late distal convoluted tubule development [GO:0072068]; is a type of metanephric nephron epithelium development [GO:0072243]; is part of metanephric distal convoluted tubule development [GO:0072221]